{
  "term_label": "regulation of transcription by RNA polymerase II",
  "gene_name": "Zinc finger X-chromosomal protein",
  "gene_symbol": "ZFX",
  "term_id": "GO:0006357",
  "gene": "UniProtKB:P17010"
}